{
  "gene": "UniProtKB:Q96BY7",
  "term_id": "GO:0061723",
  "gene_symbol": "ATG2B",
  "term_label": "glycophagy",
  "gene_name": "Autophagy-related protein 2 homolog B"
}